{
  "gene_symbol": "ITGB5",
  "term_label": "integrin-mediated signaling pathway",
  "term_id": "GO:0007229",
  "gene": "UniProtKB:P18084",
  "gene_name": "Integrin beta-5"
}